positive regulation of sporulation resulting in formation of a cellular spore [GO:0045881] (biological process) Sources: GOC:go_curators Subtypes: positive regulation of sexual sporulation resulting in formation of a cellular spore [GO:0043941], GO:0043945 Relationships: is a type of regulation of sporulation resulting in formation of a cellular spore [GO:0042173]; is a type of GO:0043938; positively regulates sporulation resulting in formation of a cellular spore [GO:0030435] Definition: Any process that activates or increases the frequency, rate or extent of sporulation. Also known as: up regulation of sporulation, up-regulation of sporulation, upregulation of sporulation, activation of sporulation, stimulation of sporulation